sulfoacetaldehyde acetyltransferase activity [GO:0050487] (molecular function) Definition: Catalysis of the reaction: acetyl phosphate + H+ + sulfite = phosphate + sulfoacetaldehyde. Sources: RHEA:24204 Also known as: sulphoacetaldehyde acetyltransferase activity, acetyl-phosphate:sulfite S-acetyltransferase (acyl-phosphate hydrolysing, 2-oxoethyl-forming) Note: The reaction occurs in the reverse direction. Relationships: is a type of acyltransferase activity, acyl groups converted into alkyl on transfer [GO:0046912]